{
  "gene": "UniProtKB:Q5SQS8",
  "term_id": "UNKNOWN:0003",
  "gene_symbol": "C10orf120",
  "term_label": "Unknown cellular component",
  "gene_name": "Uncharacterized protein C10orf120"
}